{
  "gene": "UniProtKB:A0A0A0MS00",
  "gene_symbol": "IGLV3-32",
  "term_label": "Unknown molecular function",
  "gene_name": "Probable non-functional immunoglobulin lambda variable 3-32",
  "term_id": "UNKNOWN:0001"
}